{
  "gene": "UniProtKB:Q8N9W7",
  "term_id": "UNKNOWN:0003",
  "gene_symbol": "Q8N9W7",
  "gene_name": "Putative transmembrane protein FLJ36131",
  "term_label": "Unknown cellular component"
}